positive regulation of pseudohyphal growth [GO:2000222] (biological process) Definition: Any process that activates or increases the frequency, rate or extent of pseudohyphal growth. Relationships: is a type of GO:0030307; is a type of positive regulation of growth of unicellular organism as a thread of attached cells [GO:0070786]; is a type of regulation of pseudohyphal growth [GO:2000220]; positively regulates pseudohyphal growth [GO:0007124] Sources: GOC:mah Subtypes: positive regulation of pseudohyphal growth by positive regulation of transcription from RNA polymerase II promoter [GO:1900461]